peribacteroid membrane [GO:0043661] (cellular component) Definition: A membrane that surrounds one or more bacteroids (such as nitrogen-fixing bacteroids within legume root nodule cells). Subtypes: GO:0070114 Sources: GOC:cc Relationships: is a type of endocytic vesicle membrane [GO:0030666]; is part of bacteroid-containing symbiosome [GO:0043660]